{
  "gene_symbol": "RBP2",
  "term_id": "GO:0005504",
  "term_label": "fatty acid binding",
  "gene_name": "Retinol-binding protein 2",
  "gene": "UniProtKB:P50120"
}